{
  "gene": "UniProtKB:O60231",
  "gene_name": "Pre-mRNA-splicing factor ATP-dependent RNA helicase DHX16",
  "term_id": "UNKNOWN:0002",
  "gene_symbol": "DHX16",
  "term_label": "Unknown biological process"
}